dihydrocamalexic acid decarboxylase activity [GO:0010298] (molecular function) Definition: Catalysis of the reaction: dihydrocamalexic acid = camalexin + CO2 + H+. References: PMID:16766671 Sources: MetaCyc:RXN-8275 Relationships: is a type of GO:0016831